{
  "gene": "UniProtKB:Q9UN66",
  "gene_name": "Protocadherin beta-8",
  "term_label": "cell adhesion",
  "term_id": "GO:0007155",
  "gene_symbol": "PCDHB8"
}